{
  "gene_name": "Patatin-like phospholipase domain-containing protein 2",
  "term_label": "triacylglycerol lipase activity",
  "gene": "UniProtKB:Q96AD5",
  "term_id": "GO:0004806",
  "gene_symbol": "PNPLA2"
}